{
  "gene_name": "Tyrosine-protein kinase Lyn",
  "gene": "UniProtKB:P07948",
  "term_id": "GO:0006974",
  "term_label": "DNA damage response",
  "gene_symbol": "LYN"
}